bundle of His cell to Purkinje myocyte communication by electrical coupling [GO:0086054] (biological process) Sources: GOC:BHF, GOC:mtg_cardiac_conduct_nov11 Relationships: is a type of cell communication by electrical coupling involved in cardiac conduction [GO:0086064]; is a type of GO:0086069 Definition: The process that mediates signaling interactions between a bundle of His cardiac muscle cell and a Purkinje myocyte by transfer of current between their adjacent cytoplasms via intercellular protein channels. Also known as: bundle of His cardiac muscle cell to Purkinje myocyte communication by electrical coupling